{
  "gene_name": "RCC1 and BTB domain-containing protein 1",
  "gene": "UniProtKB:Q8NDN9",
  "term_label": "Unknown molecular function",
  "gene_symbol": "RCBTB1",
  "term_id": "UNKNOWN:0001"
}